{
  "gene_symbol": "NIBAN3",
  "gene": "UniProtKB:Q86XR2",
  "term_label": "Unknown cellular component",
  "term_id": "UNKNOWN:0003",
  "gene_name": "Protein Niban 3"
}